{
  "gene_name": "Tubulin-specific chaperone A",
  "term_id": "GO:0015631",
  "gene_symbol": "TBCA",
  "term_label": "tubulin binding",
  "gene": "UniProtKB:O75347"
}